{
  "term_label": "cytosol",
  "gene_symbol": "GSTP1",
  "gene": "UniProtKB:P09211",
  "gene_name": "Glutathione S-transferase P",
  "term_id": "GO:0005829"
}